{
  "term_id": "GO:0005102",
  "term_label": "signaling receptor binding",
  "gene_name": "Ficolin-2",
  "gene": "UniProtKB:Q15485",
  "gene_symbol": "FCN2"
}